{
  "term_label": "Unknown molecular function",
  "term_id": "UNKNOWN:0001",
  "gene_symbol": "ZNF839",
  "gene": "UniProtKB:A8K0R7",
  "gene_name": "Zinc finger protein 839"
}